negative regulation of ferrichrome biosynthetic process in response to iron [GO:0097739] (biological process) Definition: Any process that stops, prevents or reduces the rate of ferrichrome biosynthetic process in response to an iron stimulus. Relationships: is a type of negative regulation of ferrichrome biosynthetic process [GO:1905569]; is part of GO:0071281 Sources: GOC:al